{
  "term_id": "GO:0031340",
  "gene_name": "Synaptotagmin-3",
  "term_label": "positive regulation of vesicle fusion",
  "gene": "UniProtKB:Q9BQG1",
  "gene_symbol": "SYT3"
}